{
  "gene_symbol": "RTKN2",
  "gene_name": "Rhotekin-2",
  "term_label": "hemopoiesis",
  "term_id": "GO:0030097",
  "gene": "UniProtKB:Q8IZC4"
}